lysosomal membrane [GO:0005765] (cellular component) Definition: The lipid bilayer surrounding the lysosome and separating its contents from the cell cytoplasm. Sources: GOC:ai Also known as: lysosome membrane Relationships: is a type of lytic vacuole membrane [GO:0098852]; is part of lysosome [GO:0005764] Subtypes: GO:0035577, endolysosome membrane [GO:0036020], phagolysosome membrane [GO:0061474], cytolytic granule membrane [GO:0101004], autolysosome membrane [GO:0120281]